{
  "term_label": "Rap protein signal transduction",
  "gene_symbol": "RAPGEF4",
  "term_id": "GO:0032486",
  "gene_name": "Rap guanine nucleotide exchange factor 4",
  "gene": "UniProtKB:Q8WZA2"
}